ent-pimara-8(14),15-diene catabolic process [GO:1901540] (biological process) Also known as: ent-pimara-8(14),15-diene breakdown, ent-pimara-8(14),15-diene catabolism, ent-pimara-8(14),15-diene degradation Sources: GOC:TermGenie, GOC:di Definition: The chemical reactions and pathways resulting in the breakdown of ent-pimara-8(14),15-diene. Relationships: is a type of terpene catabolic process [GO:0046247]